positive regulation of mesenchymal stem cell differentiation [GO:2000741] (biological process) Sources: GOC:obol Definition: Any process that activates or increases the frequency, rate or extent of mesenchymal stem cell differentiation. Relationships: is a type of positive regulation of stem cell differentiation [GO:2000738]; is a type of regulation of mesenchymal stem cell differentiation [GO:2000739]; positively regulates mesenchymal stem cell differentiation [GO:0072497] Subtypes: positive regulation of amniotic stem cell differentiation [GO:2000799]